{
  "gene_symbol": "UGT1A8",
  "term_id": "GO:0004857",
  "gene_name": "UDP-glucuronosyltransferase 1A8",
  "gene": "UniProtKB:Q9HAW9",
  "term_label": "enzyme inhibitor activity"
}